{
  "gene_name": "C-X-C chemokine receptor type 4",
  "gene": "UniProtKB:P61073",
  "term_label": "external side of plasma membrane",
  "gene_symbol": "CXCR4",
  "term_id": "GO:0009897"
}